{
  "term_label": "Unknown biological process",
  "gene_name": "Myotubularin-related protein 11",
  "term_id": "UNKNOWN:0002",
  "gene": "UniProtKB:A4FU01",
  "gene_symbol": "MTMR11"
}